{
  "gene_name": "Acyl-coenzyme A synthetase ACSM1, mitochondrial",
  "gene": "UniProtKB:Q08AH1",
  "gene_symbol": "ACSM1",
  "term_label": "acyl-CoA metabolic process",
  "term_id": "GO:0006637"
}